{
  "term_id": "GO:0003723",
  "term_label": "RNA binding",
  "gene_name": "Activating signal cointegrator 1 complex subunit 3",
  "gene_symbol": "ASCC3",
  "gene": "UniProtKB:Q8N3C0"
}